{
  "term_label": "plasma membrane",
  "term_id": "GO:0005886",
  "gene_name": "EH domain-containing protein 2",
  "gene_symbol": "EHD2",
  "gene": "UniProtKB:Q9NZN4"
}